oxidoreductase activity, acting on reduced flavodoxin as donor, dinitrogen as acceptor [GO:0016738] (molecular function) Subtypes: GO:0050142 Relationships: is a type of oxidoreductase activity, acting on reduced flavodoxin as donor [GO:0016737] Definition: Catalysis of an oxidation-reduction (redox) reaction in which reduced flavodoxin acts as a hydrogen or electron donor and reduces dinitrogen. Sources: GOC:jl